{
  "gene": "UniProtKB:Q13131",
  "term_id": "GO:0005634",
  "gene_name": "5'-AMP-activated protein kinase catalytic subunit alpha-1",
  "term_label": "nucleus",
  "gene_symbol": "PRKAA1"
}